{
  "term_id": "GO:0005737",
  "gene_symbol": "GNB4",
  "gene_name": "Guanine nucleotide-binding protein subunit beta-4",
  "term_label": "cytoplasm",
  "gene": "UniProtKB:Q9HAV0"
}